negative regulation of nervous system process [GO:0031645] (biological process) Definition: Any process that stops, prevents, or reduces the frequency, rate or extent of a neurophysiological process. Also known as: down regulation of neurological process, down-regulation of neurological process, downregulation of neurological process, negative regulation of neurological process, negative regulation of neurological system process, negative regulation of neurophysiological process, inhibition of neurological process Sources: GOC:dph, GOC:mah, GOC:tb Subtypes: negative regulation of myelination [GO:0031642], GO:0051970, GO:1904057, negative regulation of sensory perception of sweet taste [GO:1904657], GO:1904661, negative regulation of detection of mechanical stimulus involved in sensory perception of touch [GO:1905788] Relationships: is a type of GO:0031644; is a type of negative regulation of multicellular organismal process [GO:0051241]; negatively regulates GO:0050877